{
  "gene_name": "Adenomatous polyposis coli protein 2",
  "gene_symbol": "APC2",
  "term_id": "GO:0008013",
  "gene": "UniProtKB:O95996",
  "term_label": "beta-catenin binding"
}